{
  "gene_symbol": "GDI1",
  "gene": "UniProtKB:P31150",
  "term_id": "GO:0016192",
  "term_label": "vesicle-mediated transport",
  "gene_name": "Rab GDP dissociation inhibitor alpha"
}